{
  "gene_name": "Endothelial PAS domain-containing protein 1",
  "term_label": "regulation of transcription by RNA polymerase II",
  "term_id": "GO:0006357",
  "gene": "UniProtKB:Q99814",
  "gene_symbol": "EPAS1"
}